{
  "gene": "UniProtKB:Q9HBL6",
  "term_id": "UNKNOWN:0003",
  "term_label": "Unknown cellular component",
  "gene_name": "Leucine-rich repeat and transmembrane domain-containing protein 1",
  "gene_symbol": "LRTM1"
}